{
  "gene_name": "Unconventional myosin-IXb",
  "term_label": "ATP binding",
  "gene": "UniProtKB:Q13459",
  "gene_symbol": "MYO9B",
  "term_id": "GO:0005524"
}